{
  "gene_name": "Docking protein 3",
  "gene": "UniProtKB:Q7L591",
  "gene_symbol": "DOK3",
  "term_id": "GO:0035591",
  "term_label": "signaling adaptor activity"
}